{
  "gene": "UniProtKB:Q8IYA2",
  "term_id": "UNKNOWN:0002",
  "term_label": "Unknown biological process",
  "gene_name": "Putative coiled-coil domain-containing protein 144C",
  "gene_symbol": "CCDC144CP"
}